{
  "term_id": "GO:0014826",
  "gene": "UniProtKB:P20800",
  "term_label": "vein smooth muscle contraction",
  "gene_name": "Endothelin-2",
  "gene_symbol": "EDN2"
}